{
  "term_label": "cytoplasm",
  "gene_symbol": "ABHD14A",
  "term_id": "GO:0005737",
  "gene": "UniProtKB:Q9BUJ0",
  "gene_name": "Protein ABHD14A"
}